type 1 neurotensin receptor binding [GO:0031847] (MF) Sources: GOC:mah, GOC:nln Also known as: type 1 neurotensin receptor ligand Definition: Binding to a type 1 neurotensin receptor. Relationships: is a type of neurotensin receptor binding [GO:0031846]